{
  "term_id": "UNKNOWN:0001",
  "gene_symbol": "RUSF1",
  "gene": "UniProtKB:Q96GQ5",
  "term_label": "Unknown molecular function",
  "gene_name": "RUS family member 1"
}